{
  "gene_symbol": "GGPS1",
  "term_label": "isoprenoid biosynthetic process",
  "gene_name": "Geranylgeranyl pyrophosphate synthase",
  "term_id": "GO:0008299",
  "gene": "UniProtKB:O95749"
}